{
  "term_id": "GO:0005634",
  "gene_symbol": "SIM1",
  "term_label": "nucleus",
  "gene": "UniProtKB:P81133",
  "gene_name": "Single-minded homolog 1"
}